isocitrate dehydrogenase (NADP+) activity [GO:0004450] (molecular function) Also known as: NADP isocitric dehydrogenase activity, NADP(+)-linked isocitrate dehydrogenase activity, NADP-dependent isocitrate dehydrogenase activity, NADP-dependent isocitric dehydrogenase activity, NADP-linked isocitrate dehydrogenase activity, NADP-specific isocitrate dehydrogenase activity, isocitrate (NADP) dehydrogenase activity, isocitrate (nicotinamide adenine dinucleotide phosphate) dehydrogenase activity, isocitrate dehydrogenase (NADP) activity, isocitrate dehydrogenase (NADP-dependent) activity, isocitrate:NADP+ oxidoreductase (decarboxylating), triphosphopyridine nucleotide-linked isocitrate dehydrogenase activity, NADP(+)-ICDH activity, NADP(+)-IDH activity, dual-cofactor-specific isocitrate dehydrogenase activity Sources: RHEA:19629 Definition: Catalysis of the reaction: isocitrate + NADP+ = 2-oxoglutarate + CO2 + NADPH. Relationships: is a type of isocitrate dehydrogenase [NAD(P)+] activity [GO:0004448]